{
  "gene_symbol": "ADH7",
  "term_label": "retinol metabolic process",
  "term_id": "GO:0042572",
  "gene_name": "All-trans-retinol dehydrogenase [NAD(+)] ADH7",
  "gene": "UniProtKB:P40394"
}